{
  "gene": "UniProtKB:O43559",
  "gene_name": "Fibroblast growth factor receptor substrate 3",
  "term_id": "GO:0005068",
  "gene_symbol": "FRS3",
  "term_label": "transmembrane receptor protein tyrosine kinase adaptor activity"
}